{
  "gene_name": "RIB43A-like with coiled-coils protein 1",
  "gene_symbol": "RIBC1",
  "term_id": "UNKNOWN:0002",
  "term_label": "Unknown biological process",
  "gene": "UniProtKB:Q8N443"
}